positive regulation of mesoderm development [GO:2000382] (biological process) Sources: GOC:BHF Relationships: is_a GO:0051094; is a type of regulation of mesoderm development [GO:2000380]; positively regulates GO:0007498 Definition: Any process that activates or increases the frequency, rate or extent of mesoderm development. Subtypes: positive regulation of mesoderm formation [GO:1905904]